{
  "term_id": "GO:0005856",
  "gene_symbol": "TMOD1",
  "term_label": "cytoskeleton",
  "gene": "UniProtKB:P28289",
  "gene_name": "Tropomodulin-1"
}